potassium channel regulator activity [GO:0015459] (molecular function) Sources: GOC:dos, GOC:mah Subtypes: GO:0019870, GO:0099104 Also known as: potassium channel gating activity Definition: Binds to and modulates the activity of a potassium channel. Relationships: is a type of ion channel regulator activity [GO:0099106]; regulates GO:0005267